ectoine binding [GO:0033294] (molecular function) Sources: GOC:mah Relationships: is a type of monocarboxylic acid binding [GO:0033293]; is a type of heterocyclic compound binding [GO:1901363] Definition: Binding to ectoine, 1,4,5,6-tetrahydro-2-methyl-4-pyrimidinecarboxylic acid.